{
  "gene_symbol": "TBKBP1",
  "term_label": "cytoplasm",
  "term_id": "GO:0005737",
  "gene": "UniProtKB:A7MCY6",
  "gene_name": "TANK-binding kinase 1-binding protein 1"
}